{
  "term_id": "UNKNOWN:0001",
  "gene_symbol": "UGDH",
  "term_label": "Unknown molecular function",
  "gene": "UniProtKB:O60701",
  "gene_name": "UDP-glucose 6-dehydrogenase"
}